protein-lipid complex disassembly [GO:0032987] (biological process) Relationships: is a type of protein-containing complex disassembly [GO:0032984]; is a type of GO:0071825 Sources: GOC:mah Subtypes: plasma lipoprotein particle disassembly [GO:0071829] Definition: The disaggregation of a protein-lipid complex into its constituent components.